{
  "term_id": "GO:0005886",
  "term_label": "plasma membrane",
  "gene": "UniProtKB:Q03431",
  "gene_name": "Parathyroid hormone_parathyroid hormone-related peptide receptor",
  "gene_symbol": "PTH1R"
}